{
  "term_id": "GO:1901739",
  "term_label": "regulation of myoblast fusion",
  "gene": "UniProtKB:Q53GL0",
  "gene_symbol": "PLEKHO1",
  "gene_name": "Pleckstrin homology domain-containing family O member 1"
}